{
  "gene_symbol": "FANK1",
  "term_id": "GO:0005634",
  "gene_name": "Fibronectin type 3 and ankyrin repeat domains protein 1",
  "term_label": "nucleus",
  "gene": "UniProtKB:Q8TC84"
}